{
  "term_label": "Unknown molecular function",
  "gene": "UniProtKB:Q9NYS7",
  "gene_symbol": "WSB2",
  "gene_name": "WD repeat and SOCS box-containing protein 2",
  "term_id": "UNKNOWN:0001"
}